lysosomal proton-transporting V-type ATPase, V1 domain [GO:0046612] (cellular component) Definition: The V1 domain of a proton-transporting V-type ATPase found in the lysosomal membrane. Sources: GOC:mah Also known as: lysosomal hydrogen ion-transporting ATPase V1 domain Relationships: is a type of vacuolar proton-transporting V-type ATPase, V1 domain [GO:0000221]; is part of GO:0046611